{
  "gene_symbol": "MAGEB2",
  "gene_name": "Melanoma-associated antigen B2",
  "term_id": "GO:0005634",
  "gene": "UniProtKB:O15479",
  "term_label": "nucleus"
}